positive regulation of myeloid cell apoptotic process [GO:0033034] (biological process) Definition: Any process that activates or increases the frequency, rate, or extent of myeloid cell apoptotic process. Sources: GOC:add, GOC:mtg_apoptosis Also known as: up regulation of myeloid cell apoptosis, up-regulation of myeloid cell apoptosis, upregulation of myeloid cell apoptosis, activation of myeloid cell apoptosis, positive regulation of myeloid cell apoptosis, stimulation of myeloid cell apoptosis Relationships: is_a regulation of myeloid cell apoptotic process [GO:0033032]; is a type of positive regulation of apoptotic process [GO:0043065]; positively regulates myeloid cell apoptotic process [GO:0033028] Subtypes: GO:0033027, GO:0033031, positive regulation of erythrocyte apoptotic process [GO:1902252], positive regulation of macrophage apoptotic process [GO:2000111]